{
  "gene_name": "Sterol carrier protein 2",
  "gene_symbol": "SCP2",
  "gene": "UniProtKB:P22307",
  "term_label": "peroxisome",
  "term_id": "GO:0005777"
}